{
  "term_label": "plasma membrane",
  "gene_name": "Sorting nexin-18",
  "gene": "UniProtKB:Q96RF0",
  "gene_symbol": "SNX18",
  "term_id": "GO:0005886"
}